{
  "term_id": "GO:0003735",
  "term_label": "structural constituent of ribosome",
  "gene": "UniProtKB:Q6P161",
  "gene_symbol": "MRPL54",
  "gene_name": "Large ribosomal subunit protein mL54"
}